{
  "gene": "UniProtKB:P30273",
  "gene_name": "High affinity immunoglobulin epsilon receptor subunit gamma",
  "term_label": "Fc receptor mediated stimulatory signaling pathway",
  "gene_symbol": "FCER1G",
  "term_id": "GO:0002431"
}